negative regulation of appressorium formation [GO:0075019] (biological process) Also known as: negative regulation of appressorium formation on or near host Note: Note that this term should not be used to annotate gene products of the host. It should only be used to annotate those gene products from the symbiont involved in this process. Relationships: is a type of negative regulation of developmental process [GO:0051093]; is a type of regulation of appressorium formation [GO:0075017]; negatively regulates GO:0075016 Definition: Any process that stops, prevents, or reduces the frequency, rate or extent of symbiont appressorium formation. Sources: GOC:pamgo_curators